phenol O-methyltransferase activity [GO:0030736] (molecular function) Also known as: PMT, S-adenosyl-L-methionine:phenol O-methyltransferase activity Definition: Catalysis of the reaction: S-adenosyl-L-methionine + phenol = S-adenosyl-L-homocysteine + anisole + H+. Sources: EC:2.1.1.25, RHEA:14809 Relationships: is a type of GO:0008757